negative regulation of anterograde synaptic vesicle transport [GO:1903743] (biological process) Relationships: is a type of GO:1901609; is a type of negative regulation of synaptic vesicle transport [GO:1902804]; is a type of regulation of anterograde synaptic vesicle transport [GO:1903742]; negatively regulates anterograde synaptic vesicle transport [GO:0048490] References: PMID:25329901 Sources: GOC:TermGenie, GOC:kmv, GO_REF:0000058 Also known as: down regulation of anterograde synaptic vesicle transport, down-regulation of anterograde synaptic vesicle transport, downregulation of anterograde synaptic vesicle transport, inhibition of anterograde synaptic vesicle transport Definition: Any process that stops, prevents or reduces the frequency, rate or extent of anterograde synaptic vesicle transport.